{
  "gene_name": "Serine_threonine-protein phosphatase 6 regulatory ankyrin repeat subunit B",
  "gene_symbol": "ANKRD44",
  "gene": "UniProtKB:Q8N8A2",
  "term_id": "UNKNOWN:0003",
  "term_label": "Unknown cellular component"
}